{
  "gene_symbol": "RHOT2",
  "term_id": "GO:0007005",
  "gene": "UniProtKB:Q8IXI1",
  "gene_name": "Mitochondrial Rho GTPase 2",
  "term_label": "mitochondrion organization"
}